{
  "gene_symbol": "H2BC20P",
  "term_label": "nucleus",
  "gene_name": "Putative histone H2B type 2-C",
  "term_id": "GO:0005634",
  "gene": "UniProtKB:Q6DN03"
}